Scrib-APC-beta-catenin complex [GO:0034750] (cellular component) Relationships: is a type of protein-containing complex [GO:0032991]; is part of cytoplasm [GO:0005737] Definition: A protein complex that contains the Scribble protein (a cell polarity determinant), the tumor suppressor protein adenomatous polyposis coli (APC), and beta-catenin; may be involved in the control of cell proliferation. References: PMID:16611247 Note: Note that the gene/protein name 'APC' should not be confused with the abbreviation for 'anaphase promoting complex'. Also known as: hScrib-APC-beta-catenin complex